{
  "gene_symbol": "SLC25A1",
  "term_id": "GO:0071913",
  "term_label": "citrate secondary active transmembrane transporter activity",
  "gene": "UniProtKB:P53007",
  "gene_name": "Tricarboxylate transport protein, mitochondrial"
}